scyllo-inosamine-4-phosphate amidinotransferase activity [GO:0015069] (molecular function) Definition: Catalysis of the reaction: 1-amino-1-deoxy-scyllo-inositol 4-phosphate + L-arginine = 1-guanidino-1-deoxy-scyllo-inositol 4-phosphate + L-ornithine. Sources: RHEA:13265 Also known as: inosamine-phosphate amidinotransferase activity, L-arginine:1-amino-1-deoxy-scyllo-inositol-4-phosphate amidinotransferase activity, L-arginine:inosamine phosphate amidinotransferase activity, L-arginine:inosamine-P-amidinotransferase activity, inosamine-P amidinotransferase activity Relationships: is a type of GO:0015067